{
  "gene_name": "NK-tumor recognition protein",
  "gene": "UniProtKB:P30414",
  "term_label": "cyclosporin A binding",
  "term_id": "GO:0016018",
  "gene_symbol": "NKTR"
}